{
  "term_id": "GO:0004197",
  "term_label": "cysteine-type endopeptidase activity",
  "gene_name": "Cathepsin Z",
  "gene_symbol": "CTSZ",
  "gene": "UniProtKB:Q9UBR2"
}